{
  "gene_name": "Trafficking kinesin-binding protein 1",
  "term_label": "mitochondrion",
  "gene": "UniProtKB:Q9UPV9",
  "gene_symbol": "TRAK1",
  "term_id": "GO:0005739"
}